{
  "term_label": "glutamatergic synapse",
  "gene_symbol": "LRRC4",
  "term_id": "GO:0098978",
  "gene_name": "Leucine-rich repeat-containing protein 4",
  "gene": "UniProtKB:Q9HBW1"
}